{
  "term_id": "GO:0005680",
  "term_label": "anaphase-promoting complex",
  "gene": "UniProtKB:Q13042",
  "gene_symbol": "CDC16",
  "gene_name": "Cell division cycle protein 16 homolog"
}